{
  "gene_symbol": "IQCA1",
  "term_label": "microtubule severing",
  "term_id": "GO:0051013",
  "gene": "UniProtKB:Q86XH1",
  "gene_name": "Dynein regulatory complex protein 11"
}